{
  "gene_name": "Periodic tryptophan protein 2 homolog",
  "term_label": "Unknown molecular function",
  "gene": "UniProtKB:Q15269",
  "term_id": "UNKNOWN:0001",
  "gene_symbol": "PWP2"
}